{
  "gene_name": "RAC-gamma serine_threonine-protein kinase",
  "gene_symbol": "AKT3",
  "term_id": "GO:0008286",
  "term_label": "insulin receptor signaling pathway",
  "gene": "UniProtKB:Q9Y243"
}